{
  "gene": "UniProtKB:Q8WZA8",
  "gene_name": "Putative gastric cancer-related gene 224 protein",
  "term_id": "UNKNOWN:0002",
  "term_label": "Unknown biological process",
  "gene_symbol": "GCRG224"
}